{
  "term_id": "UNKNOWN:0001",
  "term_label": "Unknown molecular function",
  "gene_symbol": "LRRCC1",
  "gene_name": "Leucine-rich repeat and coiled-coil domain-containing protein 1",
  "gene": "UniProtKB:Q9C099"
}